{
  "gene_symbol": "SERPINB2",
  "gene_name": "Plasminogen activator inhibitor 2",
  "term_label": "extracellular space",
  "term_id": "GO:0005615",
  "gene": "UniProtKB:P05120"
}